{
  "gene": "UniProtKB:Q8N5L8",
  "gene_symbol": "RPP25L",
  "gene_name": "Ribonuclease P protein subunit p25-like protein",
  "term_id": "GO:0003723",
  "term_label": "RNA binding"
}